{
  "gene_name": "Charged multivesicular body protein 1b",
  "term_label": "ESCRT III complex",
  "gene_symbol": "CHMP1B",
  "gene": "UniProtKB:Q7LBR1",
  "term_id": "GO:0000815"
}